{
  "term_id": "GO:0015204",
  "gene_name": "Aquaporin-7B",
  "term_label": "urea transmembrane transporter activity",
  "gene": "UniProtKB:A0A075B734",
  "gene_symbol": "AQP7B"
}